L-tyrosine transmembrane import into vacuole [GO:0090514] (biological process) Definition: The directed movement of L-tyrosine into the vacuole across the vacuolar membrane. Sources: GOC:al Relationships: is a type of tyrosine transport [GO:0015828]; is a type of amino acid transmembrane import into vacuole [GO:0032975]; is a type of L-alpha-amino acid transmembrane transport [GO:1902475]